{
  "term_label": "neuron migration",
  "gene": "UniProtKB:P78509",
  "term_id": "GO:0001764",
  "gene_symbol": "RELN",
  "gene_name": "Reelin"
}